{
  "gene_symbol": "PRB2",
  "gene_name": "Basic salivary proline-rich protein 2",
  "term_label": "Unknown molecular function",
  "gene": "UniProtKB:P02812",
  "term_id": "UNKNOWN:0001"
}